{
  "gene_name": "Interferon regulatory factor 4",
  "term_id": "GO:0002376",
  "term_label": "immune system process",
  "gene": "UniProtKB:Q15306",
  "gene_symbol": "IRF4"
}